{
  "gene_name": "Lysine-specific demethylase 7A",
  "term_label": "transcription coregulator activity",
  "gene": "UniProtKB:Q6ZMT4",
  "gene_symbol": "KDM7A",
  "term_id": "GO:0003712"
}